{
  "term_id": "GO:0012501",
  "gene_symbol": "HTRA1",
  "term_label": "programmed cell death",
  "gene": "UniProtKB:Q92743",
  "gene_name": "Serine protease HTRA1"
}